{
  "gene": "UniProtKB:Q9NSY1",
  "term_label": "AP-2 adaptor complex binding",
  "gene_symbol": "BMP2K",
  "gene_name": "BMP-2-inducible protein kinase",
  "term_id": "GO:0035612"
}